{
  "gene_symbol": "ATP5PO",
  "term_id": "UNKNOWN:0003",
  "term_label": "Unknown cellular component",
  "gene": "UniProtKB:P48047",
  "gene_name": "ATP synthase subunit O, mitochondrial"
}